{
  "gene_symbol": "TPM2",
  "gene_name": "Tropomyosin beta chain",
  "term_label": "actin filament organization",
  "term_id": "GO:0007015",
  "gene": "UniProtKB:P07951"
}